{
  "term_id": "UNKNOWN:0001",
  "gene_symbol": "TMEM106B",
  "gene_name": "Transmembrane protein 106B",
  "gene": "UniProtKB:Q9NUM4",
  "term_label": "Unknown molecular function"
}